ADP-D-ribose modification-dependent protein binding [GO:0160002] (MF) Definition: Binding to a protein upon ADP-ribosylation of the target protein. References: PMID:26673700 Relationships: is a type of modification-dependent protein binding [GO:0140030] Subtypes: mono-ADP-D-ribose modification-dependent protein binding [GO:0160003], poly-ADP-D-ribose modification-dependent protein binding [GO:0160004] Note: This term should only be used when the binding is shown to require a ADP-D-ribose post-translational modification: the interaction needs to be tested with and without the PTM. The binding does not need to be at the site of the ADP-D-ribose modification. It may be that the PTM causes a conformational change that allows binding of the protein to another region; this type of modification-dependent protein binding is valid for annotation to this term.